{
  "term_label": "plasma membrane",
  "gene_symbol": "MARCKS",
  "gene": "UniProtKB:P29966",
  "term_id": "GO:0005886",
  "gene_name": "Myristoylated alanine-rich C-kinase substrate"
}